{
  "gene_name": "Structural maintenance of chromosomes protein 1A",
  "gene": "UniProtKB:Q14683",
  "term_id": "GO:0030893",
  "term_label": "meiotic cohesin complex",
  "gene_symbol": "SMC1A"
}